nicotianamine biosynthetic process [GO:0030418] (BP) Definition: The chemical reactions and pathways resulting in the formation of nicotianamine, 2(S),3'2(S),3''(S)-N-(N-(3-amino-3-carboxypropyl)-3-amino-3-carboxypropyl)-azetidine-2-carboxylic acid. References: PMID:10069850 Sources: GOC:mah Relationships: is a type of amino acid biosynthetic process [GO:0008652]; is a type of biogenic amine biosynthetic process [GO:0042401]; is a type of tricarboxylic acid biosynthetic process [GO:0072351] Also known as: nicotianamine anabolism, nicotianamine biosynthesis, nicotianamine formation, nicotianamine synthesis